{
  "gene_name": "Prolyl 4-hydroxylase subunit alpha-2",
  "gene_symbol": "P4HA2",
  "gene": "UniProtKB:O15460",
  "term_label": "procollagen-proline 4-dioxygenase activity",
  "term_id": "GO:0004656"
}